{
  "term_id": "UNKNOWN:0002",
  "term_label": "Unknown biological process",
  "gene_name": "Transmembrane protein 156",
  "gene_symbol": "TMEM156",
  "gene": "UniProtKB:Q8N614"
}